{
  "gene_name": "Protein myomixer",
  "gene_symbol": "MYMX",
  "gene": "UniProtKB:A0A1B0GTQ4",
  "term_label": "endoplasmic reticulum membrane",
  "term_id": "GO:0005789"
}